guanyl nucleotide exchange factor inhibitor activity [GO:1990624] (molecular function) Definition: Binds to and stops, prevents or reduces the activity of a guanyl nucleotide exchange factor. Relationships: is a type of enzyme inhibitor activity [GO:0004857] References: PMID:25635048 Sources: GOC:vw